{
  "gene_name": "NADH dehydrogenase [ubiquinone] iron-sulfur protein 6, mitochondrial",
  "term_label": "Unknown molecular function",
  "term_id": "UNKNOWN:0001",
  "gene_symbol": "NDUFS6",
  "gene": "UniProtKB:O75380"
}